{
  "term_label": "Unknown cellular component",
  "term_id": "UNKNOWN:0003",
  "gene_symbol": "SREK1",
  "gene": "UniProtKB:Q8WXA9",
  "gene_name": "Splicing regulatory glutamine_lysine-rich protein 1"
}